regulation of lateral mesodermal cell fate determination [GO:0048374] (BP) Sources: GOC:jid Subtypes: GO:0048375, GO:0048376 Also known as: regulation of lateral mesoderm cell fate determination, regulation of lateral plate mesoderm cell fate determination, regulation of lateral plate mesodermal cell fate determination Definition: Any process that modulates the frequency, rate or extent of lateral mesoderm cell fate determination. Relationships: is a type of regulation of mesodermal cell fate determination [GO:0048334]; RO_0002211 GO:0048373